{
  "gene_symbol": "SESTD1",
  "term_label": "phosphatidylinositol-3-phosphate binding",
  "term_id": "GO:0032266",
  "gene": "UniProtKB:Q86VW0",
  "gene_name": "SEC14 domain and spectrin repeat-containing protein 1"
}